{
  "term_label": "mRNA binding",
  "gene_symbol": "EIF4G3",
  "term_id": "GO:0003729",
  "gene": "UniProtKB:O43432",
  "gene_name": "Eukaryotic translation initiation factor 4 gamma 3"
}